{
  "term_label": "cytoplasm",
  "gene": "UniProtKB:P68402",
  "term_id": "GO:0005737",
  "gene_symbol": "PAFAH1B2",
  "gene_name": "Platelet-activating factor acetylhydrolase IB subunit alpha2"
}